{
  "gene_name": "Mitogen-activated protein kinase 12",
  "term_label": "intracellular signal transduction",
  "gene_symbol": "MAPK12",
  "term_id": "GO:0035556",
  "gene": "UniProtKB:P53778"
}